(R)-2-hydroxy-alpha-linolenic acid biosynthetic process [GO:1902609] (biological process) References: PMID:24214535 Sources: GOC:TermGenie, GO_REF:0000068 Also known as: 2-hydroxy-octadecatrienoic acid biosynthesis, (R)-2-hydroxy-alpha-linolenic acid anabolism, (R)-2-hydroxy-alpha-linolenic acid biosynthesis, (R)-2-hydroxy-alpha-linolenic acid formation, (R)-2-hydroxy-alpha-linolenic acid synthesis Definition: The chemical reactions and pathways resulting in the formation of (R)-2-hydroxy-alpha-linolenic acid. Relationships: is a type of GO:0006636; is a type of GO:0042759